{
  "gene": "UniProtKB:A6NKD2",
  "gene_name": "Testis-specific Y-encoded protein 2",
  "term_id": "GO:0005634",
  "term_label": "nucleus",
  "gene_symbol": "TSPY2"
}